{
  "gene_symbol": "DYNC2H1",
  "gene_name": "Cytoplasmic dynein 2 heavy chain 1",
  "gene": "UniProtKB:Q8NCM8",
  "term_label": "intraciliary retrograde transport",
  "term_id": "GO:0035721"
}